{
  "gene": "UniProtKB:Q15417",
  "term_label": "actin filament binding",
  "gene_symbol": "CNN3",
  "gene_name": "Calponin-3",
  "term_id": "GO:0051015"
}